{
  "gene": "UniProtKB:P22794",
  "gene_name": "Protein EVI2A",
  "gene_symbol": "EVI2A",
  "term_id": "UNKNOWN:0003",
  "term_label": "Unknown cellular component"
}